establishment or maintenance of cytoskeleton polarity [GO:0030952] (biological process) Also known as: cytoskeleton polarization Sources: GOC:mah Relationships: is a type of cytoskeleton organization [GO:0007010]; is a type of establishment or maintenance of cell polarity [GO:0007163] Definition: Any cellular process that results in the specification, formation or maintenance of polarized cytoskeletal structures. Subtypes: establishment or maintenance of cytoskeleton polarity involved in ameboidal cell migration [GO:0003371], cytoskeleton polarization involved in growth plate cartilage chondrocyte division [GO:0003426], establishment or maintenance of actin cytoskeleton polarity [GO:0030950], GO:0030951